{
  "term_label": "Unknown biological process",
  "term_id": "UNKNOWN:0002",
  "gene_name": "Juxtaposed with another zinc finger protein 1",
  "gene": "UniProtKB:Q86VZ6",
  "gene_symbol": "JAZF1"
}